NAD-dependent protein decrotonylase activity [GO:0160011] (molecular function) Definition: Catalysis of the reaction: H2O + N6-(2E)-butenoyl-L-lysyl-[protein] + NAD+ = 2''-O-(2E)-but-2-enoyl-ADP-D-ribose + L-lysyl-[protein] + nicotinamide. Relationships: is a type of acyltransferase activity, transferring groups other than amino-acyl groups [GO:0016747] References: PMID:28497810 Subtypes: histone decrotonylase activity, NAD-dependent [GO:0160012]